chromosome, subtelomeric region [GO:0099115] (cellular component) References: PMID:18761674, PMID:22771823, PMID:26205977, PMID:7660126 Sources: GOC:mah Relationships: is a type of chromosome, telomeric region [GO:0000781] Definition: A region of the chromosome, adjacent to the telomere (on the centromeric side) that contains repetitive DNA and sometimes genes. This region is usually heterochromatin. Also known as: subtelomere, nuclear subtelomeric heterochromatin, sub-telomeric heterochromatin, subtelomeric heterochromatin